regulation of anterograde dense core granule transport [GO:1901951] (biological process) References: PMID:23358451 Sources: GOC:TermGenie, GOC:kmv Definition: Any process that modulates the frequency, rate or extent of anterograde dense core granule transport. Relationships: is a type of GO:1901608; is a type of GO:1904809; regulates GO:1990048 Subtypes: GO:1901952, positive regulation of anterograde dense core granule transport [GO:1901953]